{
  "term_label": "regulation of Notch signaling pathway",
  "term_id": "GO:0008593",
  "gene_name": "Beta-1,3-N-acetylglucosaminyltransferase manic fringe",
  "gene_symbol": "MFNG",
  "gene": "UniProtKB:O00587"
}